{
  "term_label": "visual perception",
  "gene_symbol": "ADGRV1",
  "term_id": "GO:0007601",
  "gene_name": "Adhesion G-protein coupled receptor V1",
  "gene": "UniProtKB:Q8WXG9"
}